{
  "gene_name": "Zinc finger and BTB domain-containing protein 9",
  "term_id": "GO:0000981",
  "gene_symbol": "ZBTB9",
  "gene": "UniProtKB:Q96C00",
  "term_label": "DNA-binding transcription factor activity, RNA polymerase II-specific"
}